{
  "term_id": "GO:0031012",
  "term_label": "extracellular matrix",
  "gene_name": "von Willebrand factor A domain-containing protein 1",
  "gene_symbol": "VWA1",
  "gene": "UniProtKB:Q6PCB0"
}